{
  "gene_name": "Integrator complex subunit 3",
  "term_id": "GO:0005737",
  "term_label": "cytoplasm",
  "gene": "UniProtKB:Q68E01",
  "gene_symbol": "INTS3"
}